{
  "gene_name": "Ubiquitin carboxyl-terminal hydrolase 17-like protein 21",
  "gene_symbol": "USP17L21",
  "term_label": "regulation of protein stability",
  "term_id": "GO:0031647",
  "gene": "UniProtKB:D6R901"
}